luteinizing hormone signaling pathway [GO:0042700] (biological process) Definition: A G protein-coupled receptor signaling pathway initiated by luteinizing hormone binding to its receptor on the surface of a target cell, and ending with the regulation of a downstream cellular process. Also known as: luteinizing hormone signalling pathway Sources: GOC:dph Relationships: is a type of G protein-coupled receptor signaling pathway [GO:0007186] Subtypes: luteinizing hormone signaling pathway involved in ovarian follicle development [GO:0035471]